{
  "gene": "UniProtKB:Q8NB42",
  "term_id": "GO:0005634",
  "gene_symbol": "ZNF527",
  "term_label": "nucleus",
  "gene_name": "Zinc finger protein 527"
}